{
  "gene": "UniProtKB:Q09161",
  "term_label": "regulation of mRNA processing",
  "gene_symbol": "NCBP1",
  "term_id": "GO:0050684",
  "gene_name": "Nuclear cap-binding protein subunit 1"
}